glycine transmembrane transporter activity [GO:0015187] (MF) Relationships: is a type of GO:0015175; is a type of GO:0046943; is part of glycine transport [GO:0015816] Also known as: glycine transporter activity, glycine betaine/proline porter activity, proline/glycine/betaine:hydrogen/sodium symporter activity Sources: GOC:ai Subtypes: glycine:sodium symporter activity [GO:0015375], glycine:proton antiporter activity [GO:0140799] Definition: Enables the transfer of glycine from one side of a membrane to the other. Glycine is aminoethanoic acid.